sulfite reductase complex (NADPH) [GO:0009337] (cellular component) Also known as: sulphite reductase complex (NADPH) Definition: A multisubunit iron flavoprotein, which in yeast is composed of 2 alpha and 2 beta subunits. Catalyzes the reduction of sulfite to sulfide. References: PMID:6751400 Sources: GOC:jl Note: See also the molecular function term 'sulfite reductase (NADPH) activity ; GO:0004783'. Relationships: is a type of intracellular protein-containing complex [GO:0140535]; is a type of GO:1902494